{
  "gene_symbol": "KLHL28",
  "term_id": "GO:0043161",
  "term_label": "proteasome-mediated ubiquitin-dependent protein catabolic process",
  "gene": "UniProtKB:Q9NXS3",
  "gene_name": "Kelch-like protein 28"
}